{
  "gene_symbol": "MTRR",
  "gene": "UniProtKB:Q9UBK8",
  "term_label": "flavin adenine dinucleotide binding",
  "term_id": "GO:0050660",
  "gene_name": "Methionine synthase reductase"
}